{
  "gene": "UniProtKB:P07948",
  "term_id": "GO:0002431",
  "term_label": "Fc receptor mediated stimulatory signaling pathway",
  "gene_name": "Tyrosine-protein kinase Lyn",
  "gene_symbol": "LYN"
}